epicuticle of collagen and cuticulin-based cuticle extracellular matrix [GO:0060105] (CC) Also known as: epicuticle of collagen and cuticulin-based exoskeleton extracellular matrix Relationships: is a type of cellular anatomical structure [GO:0110165]; is part of cuticular extracellular matrix [GO:0060102] Definition: A lipid-containing layer of cuticle that lies between the cortical layer and the surface coat. An example of this component is found in Caenorhabditis elegans. Sources: GOC:dph, GOC:kmv, ISSN:15518507